{
  "gene_name": "Prefoldin subunit 6",
  "term_label": "chaperone-mediated protein complex assembly",
  "gene": "UniProtKB:O15212",
  "term_id": "GO:0051131",
  "gene_symbol": "PFDN6"
}